{
  "term_label": "NADH dehydrogenase activity",
  "gene": "UniProtKB:O00217",
  "gene_symbol": "NDUFS8",
  "gene_name": "NADH dehydrogenase [ubiquinone] iron-sulfur protein 8, mitochondrial",
  "term_id": "GO:0003954"
}